{
  "gene_name": "Chloride intracellular channel protein 4",
  "gene_symbol": "CLIC4",
  "term_id": "GO:0006821",
  "gene": "UniProtKB:Q9Y696",
  "term_label": "chloride transport"
}